{
  "gene": "UniProtKB:Q9UBX3",
  "term_id": "GO:0005743",
  "gene_symbol": "SLC25A10",
  "gene_name": "Mitochondrial dicarboxylate carrier",
  "term_label": "mitochondrial inner membrane"
}